{
  "term_id": "GO:0050727",
  "gene_symbol": "AHSG",
  "gene_name": "Alpha-2-HS-glycoprotein",
  "gene": "UniProtKB:P02765",
  "term_label": "regulation of inflammatory response"
}